{
  "gene": "UniProtKB:Q12834",
  "term_label": "ubiquitin ligase activator activity",
  "term_id": "GO:1990757",
  "gene_symbol": "CDC20",
  "gene_name": "Cell division cycle protein 20 homolog"
}